{
  "gene": "UniProtKB:P17342",
  "gene_symbol": "NPR3",
  "term_label": "peptide hormone binding",
  "term_id": "GO:0017046",
  "gene_name": "Atrial natriuretic peptide receptor 3"
}